{
  "gene": "UniProtKB:Q9Y284",
  "gene_name": "PAT complex subunit Asterix",
  "gene_symbol": "WDR83OS",
  "term_id": "GO:0005789",
  "term_label": "endoplasmic reticulum membrane"
}